{
  "term_label": "negative regulation of G protein-coupled receptor signaling pathway",
  "term_id": "GO:0045744",
  "gene_name": "Regulator of G-protein signaling 20",
  "gene": "UniProtKB:O76081",
  "gene_symbol": "RGS20"
}